{
  "term_id": "GO:0042393",
  "gene_name": "Bromodomain-containing protein 2",
  "gene": "UniProtKB:P25440",
  "gene_symbol": "BRD2",
  "term_label": "histone binding"
}